{
  "term_id": "GO:0004123",
  "gene_symbol": "CTH",
  "term_label": "cystathionine gamma-lyase activity",
  "gene_name": "Cystathionine gamma-lyase",
  "gene": "UniProtKB:P32929"
}